negative regulation of DNA catabolic process [GO:1903625] (biological process) Definition: Any process that stops, prevents or reduces the frequency, rate or extent of DNA catabolic process. References: PMID:2001740 Sources: GOC:TermGenie, GO_REF:0000058 Also known as: down regulation of DNA breakdown, down regulation of DNA catabolic process, down regulation of DNA catabolism, down regulation of DNA degradation, down-regulation of DNA breakdown, down-regulation of DNA catabolic process, down-regulation of DNA catabolism, down-regulation of DNA degradation, downregulation of DNA breakdown, downregulation of DNA catabolic process, downregulation of DNA catabolism, downregulation of DNA degradation, negative regulation of DNA breakdown, negative regulation of DNA catabolism, negative regulation of DNA degradation, inhibition of DNA breakdown, inhibition of DNA catabolic process, inhibition of DNA catabolism, inhibition of DNA degradation Relationships: is a type of GO:0009895; is a type of negative regulation of DNA metabolic process [GO:0051053]; is a type of regulation of DNA catabolic process [GO:1903624]; negatively regulates DNA catabolic process [GO:0006308] Subtypes: negative regulation of apoptotic DNA fragmentation [GO:1902511]